{
  "gene_symbol": "ACP5",
  "term_label": "ferric iron binding",
  "gene_name": "Tartrate-resistant acid phosphatase type 5",
  "term_id": "GO:0008199",
  "gene": "UniProtKB:P13686"
}